{
  "gene_symbol": "EID3",
  "gene": "UniProtKB:Q8N140",
  "term_label": "DNA repair",
  "gene_name": "EP300-interacting inhibitor of differentiation 3",
  "term_id": "GO:0006281"
}